negative regulation of inclusion body assembly [GO:0090084] (biological process) Definition: Any process that decreases the rate, frequency, or extent of inclusion body assembly. Inclusion body assembly is the aggregation, arrangement and bonding together of a set of components to form an inclusion body. Subtypes: negative regulation of Lewy body formation [GO:0140123], negative regulation of neurofibrillary tangle assembly [GO:1902997] Sources: GOC:BHF, GOC:dph, GOC:tb Relationships: is a type of GO:0051129; is a type of regulation of inclusion body assembly [GO:0090083]; negatively regulates inclusion body assembly [GO:0070841]